{
  "term_id": "UNKNOWN:0002",
  "gene_name": "Nucleolar RNA helicase 2",
  "term_label": "Unknown biological process",
  "gene_symbol": "DDX21",
  "gene": "UniProtKB:Q9NR30"
}